{
  "term_id": "UNKNOWN:0001",
  "gene_symbol": "MACIR",
  "gene": "UniProtKB:Q96GV9",
  "gene_name": "Macrophage immunometabolism regulator",
  "term_label": "Unknown molecular function"
}